bone trabecula morphogenesis [GO:0061430] (biological process) Relationships: is a type of GO:0061383 Definition: The process of shaping a trabecula in bone. A trabecula is a tissue element in the form of a small beam, strut or rod. Sources: GOC:BHF, GOC:dph, GOC:vk